{
  "term_id": "UNKNOWN:0002",
  "gene_name": "Atos homolog protein B",
  "term_label": "Unknown biological process",
  "gene_symbol": "ATOSB",
  "gene": "UniProtKB:Q7L5A3"
}